{
  "term_label": "negative regulation of DNA-templated transcription",
  "gene_symbol": "SPINDOC",
  "term_id": "GO:0045892",
  "gene_name": "Spindlin interactor and repressor of chromatin-binding protein",
  "gene": "UniProtKB:Q9BUA3"
}